5-guanidino-2-oxopentanoate decarboxylase activity [GO:0047435] (molecular function) Relationships: is a type of carboxy-lyase activity [GO:0016831] Also known as: 2-oxo-5-guanidinopentanoate carboxy-lyase (4-guanidinobutanal-forming), 2-oxo-5-guanidinopentanoate carboxy-lyase activity, 2-oxo-5-guanidinopentanoate decarboxylase activity, 2-oxo-5-guanidinovalerate alpha-ketoarginine decarboxylase activity, alpha-ketoarginine decarboxylase activity Definition: Catalysis of the reaction: 5-guanidino-2-oxopentanoate + H+ = 4-guanidinobutanal + CO2. Sources: EC:4.1.1.75, RHEA:11340